{
  "term_label": "kinetochore",
  "gene": "UniProtKB:P33981",
  "gene_name": "Dual specificity protein kinase TTK",
  "gene_symbol": "TTK",
  "term_id": "GO:0000776"
}